type III protein secretion system complex [GO:0030257] (cellular component) References: PMID:9618447 Definition: A complex of approximately 20 proteins, most of which are located in the cytoplasmic membrane that carries out protein secretion in the bacterial type III secretion system; type III secretion also requires a cytoplasmic, probably membrane-associated ATPase. Also known as: T3SS complex, TTSS complex Relationships: is a type of GO:0032991